adventurous gliding motility [GO:0030982] (biological process) Definition: A process involved in the controlled movement of a bacterial cell powered by the rearward secretion of carbohydrate slime. Relationships: is a type of cell gliding [GO:0071976] References: PMID:11967173 Sources: GOC:mlg Also known as: adventurous gliding movement